{
  "term_label": "programmed cell death",
  "gene_name": "Serine protease HTRA2, mitochondrial",
  "term_id": "GO:0012501",
  "gene_symbol": "HTRA2",
  "gene": "UniProtKB:O43464"
}